{
  "gene": "UniProtKB:P19622",
  "term_id": "GO:0005634",
  "gene_symbol": "EN2",
  "gene_name": "Homeobox protein engrailed-2",
  "term_label": "nucleus"
}